negative regulation of eosinophil extravasation [GO:2000420] (biological process) Relationships: is a type of negative regulation of cellular extravasation [GO:0002692]; is a type of negative regulation of eosinophil migration [GO:2000417]; is a type of regulation of eosinophil extravasation [GO:2000419]; negatively regulates eosinophil extravasation [GO:0072682] Definition: Any process that stops, prevents or reduces the frequency, rate or extent of eosinophil extravasation. Sources: GOC:BHF, GOC:mah